anterior/posterior pattern specification involved in pronephros development [GO:0034672] (biological process) Definition: The developmental process that results in the creation of defined areas or spaces within the pronephros along the anterior/posterior axis to which cells respond and eventually are instructed to differentiate. Also known as: anterior/posterior pattern specification involved in pronephric kidney development Relationships: is a type of GO:0039017; is a type of anterior/posterior pattern specification involved in kidney development [GO:0072098] Sources: GOC:mah